{
  "term_id": "GO:0048870",
  "gene_name": "Protein LRATD1",
  "gene": "UniProtKB:Q96KN4",
  "gene_symbol": "LRATD1",
  "term_label": "cell motility"
}